{
  "gene": "UniProtKB:Q8IZM8",
  "term_id": "GO:0006357",
  "gene_symbol": "ZNF654",
  "term_label": "regulation of transcription by RNA polymerase II",
  "gene_name": "Zinc finger protein 654"
}